{
  "gene": "UniProtKB:O43704",
  "term_id": "GO:0005737",
  "gene_symbol": "SULT1B1",
  "term_label": "cytoplasm",
  "gene_name": "Sulfotransferase 1B1"
}